{
  "gene_symbol": "EBF3",
  "gene_name": "Transcription factor COE3",
  "term_id": "GO:0000978",
  "term_label": "RNA polymerase II cis-regulatory region sequence-specific DNA binding",
  "gene": "UniProtKB:Q9H4W6"
}